{
  "gene_symbol": "PNMA8C",
  "gene_name": "Paraneoplastic antigen-like protein 8C",
  "gene": "UniProtKB:A0A1B0GUJ8",
  "term_label": "Unknown cellular component",
  "term_id": "UNKNOWN:0003"
}